{
  "term_id": "GO:0008045",
  "gene": "UniProtKB:P51805",
  "term_label": "motor neuron axon guidance",
  "gene_name": "Plexin-A3",
  "gene_symbol": "PLXNA3"
}